{
  "gene_name": "Protein FAM246B",
  "gene_symbol": "FAM246B",
  "gene": "UniProtKB:A0A494C0N9",
  "term_id": "UNKNOWN:0003",
  "term_label": "Unknown cellular component"
}